follicular dendritic cell activation involved in immune response [GO:0002267] (biological process) Definition: A change in the morphology or behavior of a follicular dendritic cell resulting from exposure to an activating factor such as a cellular or soluble ligand, leading to the initiation or perpetuation of an immune response. References: PMID:15606789 Sources: GOC:add Relationships: is a type of cell activation involved in immune response [GO:0002263]; is a type of GO:0002266 Also known as: follicular dendritic cell activation during immune response